N-methylhydantoinase (ATP-hydrolyzing) activity [GO:0047423] (MF) Sources: EC:3.5.2.14, RHEA:11720 Definition: Catalysis of the reaction: N-methylhydantoin + ATP + 2 H2O = N-carbamoylsarcosine + ADP + 3 H+ + phosphate. Relationships: is a type of hydrolase activity, acting on carbon-nitrogen (but not peptide) bonds, in cyclic amides [GO:0016812] Also known as: N-methylhydantoin amidohydrolase activity, N-methylhydantoin hydrolase activity, N-methylhydantoinase (ATP-hydrolysing), N-methylhydantoinase activity, N-methylimidazolidine-2,4-dione amidohydrolase (ATP-hydrolysing), methylhydantoin amidase activity